positive regulation of antimicrobial humoral response [GO:0002760] (biological process) Sources: GOC:add Relationships: is a type of regulation of antimicrobial humoral response [GO:0002759]; is a type of positive regulation of response to biotic stimulus [GO:0002833]; is a type of GO:0002922; is a type of GO:0031349; is a type of positive regulation of response to external stimulus [GO:0032103]; positively regulates GO:0019730 Definition: Any process that activates or increases the frequency, rate, or extent of an antimicrobial humoral response. Subtypes: GO:0002225 Also known as: up regulation of antimicrobial humoral response, up-regulation of antimicrobial humoral response, upregulation of antimicrobial humoral response, activation of antimicrobial humoral response, stimulation of antimicrobial humoral response